{
  "term_label": "SCF-dependent proteasomal ubiquitin-dependent protein catabolic process",
  "gene_name": "F-box_LRR-repeat protein 14",
  "gene": "UniProtKB:Q8N1E6",
  "term_id": "GO:0031146",
  "gene_symbol": "FBXL14"
}